{
  "term_label": "serine-type endopeptidase inhibitor activity",
  "gene_name": "Alpha-1-antichymotrypsin",
  "gene": "UniProtKB:P01011",
  "gene_symbol": "SERPINA3",
  "term_id": "GO:0004867"
}